{
  "gene_name": "Protein unc-13 homolog B",
  "term_label": "synaptic vesicle membrane",
  "term_id": "GO:0030672",
  "gene_symbol": "UNC13B",
  "gene": "UniProtKB:O14795"
}